positive regulation of glutamate neurotransmitter secretion in response to membrane depolarization [GO:0061646] (BP) Relationships: is a type of cellular response to stimulus [GO:0051716]; is a type of GO:1903296 Definition: Any process that activates or increases the frequency, rate or extent of glutamate secretion in response to membrane depolarization, where glutamate acts as a neurotransmitter. Sources: GOC:PARL, GOC:pad